{
  "term_label": "hydrogen peroxide catabolic process",
  "term_id": "GO:0042744",
  "gene_symbol": "PRDX2",
  "gene": "UniProtKB:P32119",
  "gene_name": "Peroxiredoxin-2"
}